{
  "gene_name": "Glutathione hydrolase 5 proenzyme",
  "gene": "UniProtKB:P36269",
  "gene_symbol": "GGT5",
  "term_label": "inflammatory response",
  "term_id": "GO:0006954"
}